positive regulation of heart rate by epinephrine [GO:0003065] (biological process) Definition: The process in which the secretion of epinephrine into the bloodstream or released from nerve endings increases the rate of heart muscle contraction. Also known as: adrenaline cardiac chronotropy, adrenaline regulation of the rate of heart muscle contraction, epinephrine cardiac chronotropy, positive regulation of heart contraction rate by epinephrine, positive regulation of heart rate by adrenaline Relationships: is a type of GO:0003062; is a type of positive regulation of heart rate [GO:0010460]; is part of positive regulation of heart rate by epinephrine-norepinephrine [GO:0001996] Sources: GOC:mtg_cardio, GOC:rl Subtypes: GO:0003111, positive regulation of heart rate by neuronal epinephrine [GO:0003112]